cadmium ion sensor activity [GO:0097063] (molecular function) References: PMID:19456862 Sources: GOC:rs Relationships: is a type of metal ion sensor activity [GO:0140784]; has part cadmium ion binding [GO:0046870] Definition: Binding to and responding, e.g. by conformational change, to changes in the cellular level of cadmium (Cd++).